{
  "gene_name": "Phosphatidylinositol transfer protein alpha isoform",
  "term_id": "GO:0008525",
  "gene_symbol": "PITPNA",
  "gene": "UniProtKB:Q00169",
  "term_label": "phosphatidylcholine transporter activity"
}